{
  "gene": "UniProtKB:Q16082",
  "term_id": "GO:0042026",
  "gene_symbol": "HSPB2",
  "term_label": "protein refolding",
  "gene_name": "Heat shock protein beta-2"
}